{
  "term_id": "GO:0007052",
  "gene_symbol": "PLK1",
  "gene_name": "Serine_threonine-protein kinase PLK1",
  "gene": "UniProtKB:P53350",
  "term_label": "mitotic spindle organization"
}